{
  "gene_name": "Coiled-coil domain-containing protein 160",
  "term_label": "Unknown cellular component",
  "gene_symbol": "CCDC160",
  "gene": "UniProtKB:A6NGH7",
  "term_id": "UNKNOWN:0003"
}